L-cystine L-cysteine-lyase (deaminating) [GO:0044540] (molecular function) Relationships: is a type of carbon-sulfur lyase activity [GO:0016846] Definition: Catalysis of the reaction: L-cystine + H2O = pyruvate + NH3 + thiocysteine. Thiocysteine is also known as cysteine persulfide. Sources: GOC:jl, RHEA:24927